{
  "gene": "UniProtKB:A0A087WSZ9",
  "term_id": "GO:0009617",
  "gene_symbol": "TRAV30",
  "gene_name": "T cell receptor alpha variable 30",
  "term_label": "response to bacterium"
}